{
  "term_label": "intracellular zinc ion homeostasis",
  "gene_symbol": "SLC30A10",
  "gene": "UniProtKB:Q6XR72",
  "term_id": "GO:0006882",
  "gene_name": "Calcium_manganese antiporter SLC30A10"
}